regulation of toll-like receptor 12 signaling pathway [GO:0034175] (biological process) Subtypes: GO:0034176, positive regulation of toll-like receptor 12 signaling pathway [GO:0034177] References: PMID:16551253, PMID:17328678 Sources: GOC:add Definition: Any process that modulates the frequency, rate, or extent of toll-like receptor 12 signaling pathway. Relationships: is a type of regulation of cytoplasmic pattern recognition receptor signaling pathway [GO:0039531]; regulates toll-like receptor 12 signaling pathway [GO:0034174] Also known as: regulation of TLR12 signaling pathway, regulation of toll-like receptor 12 signalling pathway